{
  "gene_symbol": "GIMAP4",
  "gene_name": "GTPase IMAP family member 4",
  "term_label": "GTPase activity",
  "term_id": "GO:0003924",
  "gene": "UniProtKB:Q9NUV9"
}